polytene chromosome puffing [GO:0035079] (biological process) Subtypes: ecdysone-mediated polytene chromosome puffing [GO:0035077], heat shock-mediated polytene chromosome puffing [GO:0035080] Relationships: is a type of chromosome organization [GO:0051276] References: PMID:12543962 Sources: GOC:bf Definition: The decondensing (loosening) and swelling of the chromosomal sites of target genes on polytene chromosomes following response to a stimulus, to facilitate sudden bursts of transcriptional activity in response to transient environmental signals.